{
  "gene_name": "NADH dehydrogenase [ubiquinone] 1 beta subcomplex subunit 1",
  "term_label": "Unknown biological process",
  "term_id": "UNKNOWN:0002",
  "gene_symbol": "NDUFB1",
  "gene": "UniProtKB:O75438"
}